platelet SNARE complex [GO:0097654] (cellular component) References: PMID:12130530, PMID:19450911 Sources: GOC:bhm Relationships: is a type of GO:0031201 Definition: A SNARE complex that is capable of fusing intracellular vesicles to the plasma membrane of platelets for exocytosis of alpha-granules or dense granules. Contains isoforms of VAMP, SNAP and syntaxin proteins. Ternary SNARE complexes interact in a circular array to form ring complexes or channels around the membrane fusion. A common composition in human is VAMP-8, SNAP-23 and syntaxin-2 or -4.